{
  "gene_symbol": "PIK3C3",
  "gene_name": "Phosphatidylinositol 3-kinase catalytic subunit type 3",
  "term_id": "GO:0000407",
  "gene": "UniProtKB:Q8NEB9",
  "term_label": "phagophore assembly site"
}